{
  "gene_name": "Mitochondrial protein C2orf69",
  "term_label": "mitochondrion",
  "term_id": "GO:0005739",
  "gene": "UniProtKB:Q8N8R5",
  "gene_symbol": "C2orf69"
}